{
  "term_id": "GO:0034704",
  "gene_symbol": "RYR3",
  "term_label": "calcium channel complex",
  "gene_name": "Ryanodine receptor 3",
  "gene": "UniProtKB:Q15413"
}